protein localization to subtelomeric heterochromatin [GO:1903213] (BP) References: PMID:21300781 Sources: GOC:TermGenie, GO_REF:0000087, SO:0001997 Relationships: is a type of protein localization to chromosome, telomeric region [GO:0070198]; is a type of protein localization to heterochromatin [GO:0097355] Definition: A process in which a protein is transported to, or maintained in, a location within a subtelomeric heterochromatin. Also known as: protein localisation in subtelomeric heterochromatin, protein localisation to subtelomeric heterochromatin, protein localization in subtelomeric heterochromatin, protein localisation to telomeric heterochromatin, protein localization to telomeric heterochromatin